glutamate dehydrogenase [NAD(P)+] activity [GO:0004353] (molecular function) Relationships: is a type of oxidoreductase activity, acting on the CH-NH2 group of donors, NAD or NADP as acceptor [GO:0016639] Note: Note that this term has a MetaCyc pathway reference as the pathway only has a single step. Also known as: glutamic dehydrogenase activity, L-glutamate:NAD(P)+ oxidoreductase (deaminating), glutamate biosynthesis, using glutamate dehydrogenase (NAD(P)+), glutamate biosynthetic process, using glutamate dehydrogenase (NAD(P)+) Definition: Catalysis of the reaction: L-glutamate + H2O + NAD(P)+ = 2-oxoglutarate + NH3 + NAD(P)H + H+. Sources: EC:1.4.1.3 Subtypes: glutamate dehydrogenase (NAD+) activity [GO:0004352], glutamate dehydrogenase (NADP+) activity [GO:0004354]